{
  "term_label": "cytoplasm",
  "gene_name": "Casein kinase I isoform gamma-2",
  "gene_symbol": "CSNK1G2",
  "gene": "UniProtKB:P78368",
  "term_id": "GO:0005737"
}